{
  "term_label": "embryonic organ development",
  "gene": "UniProtKB:P19447",
  "gene_name": "General transcription and DNA repair factor IIH helicase subunit XPB",
  "term_id": "GO:0048568",
  "gene_symbol": "ERCC3"
}